{
  "term_id": "GO:0042110",
  "gene": "UniProtKB:Q9HBG7",
  "gene_symbol": "LY9",
  "term_label": "T cell activation",
  "gene_name": "T-lymphocyte surface antigen Ly-9"
}